{
  "gene_name": "Ran GTPase-activating protein 1",
  "gene_symbol": "RANGAP1",
  "gene": "UniProtKB:P46060",
  "term_id": "GO:0031267",
  "term_label": "small GTPase binding"
}